{
  "term_id": "UNKNOWN:0001",
  "term_label": "Unknown molecular function",
  "gene_name": "Probable non-functional immunoglobulin kappa variable 1D-42",
  "gene_symbol": "IGKV1D-42",
  "gene": "UniProtKB:A0A075B6H8"
}